{
  "gene": "UniProtKB:A0AVI4",
  "gene_name": "E3 ubiquitin-protein ligase TM129",
  "term_id": "GO:0005783",
  "gene_symbol": "TMEM129",
  "term_label": "endoplasmic reticulum"
}